{
  "gene_symbol": "C10orf53",
  "gene_name": "UPF0728 protein C10orf53",
  "term_label": "Unknown molecular function",
  "gene": "UniProtKB:Q8N6V4",
  "term_id": "UNKNOWN:0001"
}